{
  "term_id": "GO:0005634",
  "gene_symbol": "NCBP3",
  "gene_name": "Nuclear cap-binding protein subunit 3",
  "term_label": "nucleus",
  "gene": "UniProtKB:Q53F19"
}